{
  "term_label": "midbody",
  "gene_symbol": "KLHDC8B",
  "gene_name": "Kelch domain-containing protein 8B",
  "gene": "UniProtKB:Q8IXV7",
  "term_id": "GO:0030496"
}